hydroquinone glucosyltransferase activity [GO:0050505] (molecular function) Definition: Catalysis of the reaction: hydroquinone + UDP-D-glucose = H+ + hydroquinone O-beta-D-glucopyranoside + UDP. Sources: EC:2.4.1.218, RHEA:12560 Also known as: UDP-glucose:hydroquinone-O-beta-D-glucosyltransferase activity, UDPglucose:hydroquinone-O-beta-D-glucosyltransferase activity, arbutin synthase activity, hydroquinone:O-glucosyltransferase activity Relationships: is a type of GO:0035251